{
  "gene": "UniProtKB:A0PJE2",
  "term_id": "UNKNOWN:0001",
  "term_label": "Unknown molecular function",
  "gene_symbol": "DHRS12",
  "gene_name": "Dehydrogenase_reductase SDR family member 12"
}